{
  "term_id": "UNKNOWN:0002",
  "gene": "UniProtKB:Q9C098",
  "gene_name": "Serine_threonine-protein kinase DCLK3",
  "gene_symbol": "DCLK3",
  "term_label": "Unknown biological process"
}